{
  "gene_name": "(E2-independent) E3 ubiquitin-conjugating enzyme FATS",
  "gene_symbol": "C10orf90",
  "gene": "UniProtKB:Q96M02",
  "term_label": "centriole",
  "term_id": "GO:0005814"
}